{
  "gene_name": "Coagulation factor XII",
  "gene_symbol": "F12",
  "gene": "UniProtKB:P00748",
  "term_label": "extracellular space",
  "term_id": "GO:0005615"
}